{
  "term_id": "GO:0006212",
  "gene_symbol": "DPYD",
  "gene": "UniProtKB:Q12882",
  "gene_name": "Dihydropyrimidine dehydrogenase [NADP(+)]",
  "term_label": "uracil catabolic process"
}